benzene 1,2-dioxygenase activity [GO:0018619] (molecular function) Relationships: is a type of oxidoreductase activity, acting on paired donors, with incorporation or reduction of molecular oxygen, NAD(P)H as one donor, and incorporation of two atoms of oxygen into one donor [GO:0016708] Definition: Catalysis of the reaction: benzene + H+ + NADH + O2 = cis-cyclohexa-3,5-diene-1,2-diol + NAD+. Sources: EC:1.14.12.3, RHEA:13813 Also known as: benzene dioxygenase activity, benzene hydroxylase activity, benzene,NADH:oxygen oxidoreductase (1,2-hydroxylating)